{
  "gene_name": "Nucleolar MIF4G domain-containing protein 1",
  "gene": "UniProtKB:Q5C9Z4",
  "gene_symbol": "NOM1",
  "term_id": "GO:0003723",
  "term_label": "RNA binding"
}